{
  "term_id": "GO:0071962",
  "gene": "UniProtKB:Q562F6",
  "gene_name": "Shugoshin 2",
  "gene_symbol": "SGO2",
  "term_label": "mitotic sister chromatid cohesion, centromeric"
}